{
  "term_id": "GO:0003724",
  "gene_name": "Probable ATP-dependent RNA helicase DDX4",
  "gene": "UniProtKB:Q9NQI0",
  "gene_symbol": "DDX4",
  "term_label": "RNA helicase activity"
}